{
  "term_id": "UNKNOWN:0002",
  "gene_name": "Endoplasmic reticulum membrane-associated RNA degradation protein",
  "gene": "UniProtKB:Q5T6L9",
  "gene_symbol": "ERMARD",
  "term_label": "Unknown biological process"
}